{
  "term_id": "GO:0000981",
  "gene_name": "Musculin",
  "term_label": "DNA-binding transcription factor activity, RNA polymerase II-specific",
  "gene_symbol": "MSC",
  "gene": "UniProtKB:O60682"
}